{
  "term_id": "GO:0004503",
  "term_label": "tyrosinase activity",
  "gene_symbol": "TYRP1",
  "gene_name": "5,6-dihydroxyindole-2-carboxylic acid oxidase",
  "gene": "UniProtKB:P17643"
}